RNA surveillance [GO:0071025] (biological process) Subtypes: cytoplasmic RNA surveillance [GO:0071026], GO:0071027, tRNA surveillance [GO:0106354] Relationships: is a type of GO:0006401 References: PMID:18644474 Sources: GOC:dgf, GOC:krc Definition: A process that identifies and degrades defective or aberrant RNAs. Also known as: RNA quality control, aberrant RNA catabolic process